{
  "gene": "UniProtKB:P48546",
  "gene_symbol": "GIPR",
  "term_label": "peptide hormone binding",
  "term_id": "GO:0017046",
  "gene_name": "Gastric inhibitory polypeptide receptor"
}